{
  "term_id": "GO:0099536",
  "gene_symbol": "UTRN",
  "term_label": "synaptic signaling",
  "gene_name": "Utrophin",
  "gene": "UniProtKB:P46939"
}